{
  "term_label": "structural constituent of ribosome",
  "term_id": "GO:0003735",
  "gene_name": "Small ribosomal subunit protein uS2m",
  "gene_symbol": "MRPS2",
  "gene": "UniProtKB:Q9Y399"
}